{
  "term_id": "GO:0009954",
  "term_label": "proximal/distal pattern formation",
  "gene_name": "Homeobox protein Hox-B9",
  "gene": "UniProtKB:P17482",
  "gene_symbol": "HOXB9"
}